{
  "term_label": "Unknown molecular function",
  "gene_symbol": "FAM149A",
  "gene": "UniProtKB:A5PLN7",
  "term_id": "UNKNOWN:0001",
  "gene_name": "Protein FAM149A"
}